regulation of apoptosome assembly [GO:1905100] (biological process) Also known as: regulation of apoptosome formation Relationships: is a type of regulation of protein-containing complex assembly [GO:0043254]; regulates apoptosome assembly [GO:0097314] Subtypes: negative regulation of apoptosome assembly [GO:1905101], positive regulation of apoptosome assembly [GO:1905102] Definition: Any process that modulates the frequency, rate or extent of apoptosome assembly. References: PMID:26265044 Sources: GOC:BHF, GOC:BHF_miRNA, GOC:TermGenie, GOC:bc, GO_REF:0000058